regulation of compound eye retinal cell apoptotic process [GO:1901692] (BP) Definition: Any process that modulates the frequency, rate or extent of compound eye retinal cell apoptotic process. Subtypes: negative regulation of compound eye retinal cell apoptotic process [GO:1901693], GO:1901694 References: PMID:12021768 Sources: GOC:TermGenie, GOC:mtg_apoptosis Relationships: is_a regulation of apoptotic process [GO:0042981]; regulates GO:1990010